spindle pole body-nuclear membrane anchor activity [GO:0106166] (molecular function) Definition: The binding activity of a molecule that brings together a mitotic spindle pole body and the nuclear membrane, in order to maintain specific membrane location of the spindle pole body. Relationships: is a type of protein-membrane adaptor activity [GO:0043495]; is a type of spindle pole body anchor activity [GO:0140475] References: PMID:9763447 Sources: GOC:vw Also known as: nuclear membrane-spindle pole body anchor activity, spindle pole body nuclear membrane anchor activity